{
  "term_label": "glutathione transferase activity",
  "gene_symbol": "GSTTP2",
  "gene_name": "glutathione transferase",
  "term_id": "GO:0004364",
  "gene": "UniProtKB:A0A1W2PRG0"
}